positive regulation of amine transport [GO:0051954] (biological process) Also known as: up regulation of amine transport, up-regulation of amine transport, upregulation of amine transport, activation of amine transport, stimulation of amine transport Sources: GOC:ai Definition: Any process that activates, maintains or increases the frequency, rate or extent of the directed movement of amines into, out of or within a cell, or between cells, by means of some agent such as a transporter or pore. Subtypes: GO:0014057, positive regulation of catecholamine secretion [GO:0033605], GO:0051633, positive regulation of catecholamine uptake involved in synaptic transmission [GO:0051944], GO:0051957 Relationships: is a type of positive regulation of transport [GO:0051050]; is a type of regulation of amine transport [GO:0051952]; positively regulates amine transport [GO:0015837]